alpha-ketoglutarate:proton symporter activity [GO:0015532] (molecular function) Relationships: is a type of alpha-ketoglutarate transmembrane transporter activity [GO:0015139]; is a type of GO:0015295 Sources: TC:2.A.1.6.2 Definition: Enables the transfer of a solute or solutes from one side of a membrane to the other according to the reaction: alpha-ketoglutarate(out) + H+(out) = alpha-ketoglutarate(in) + H+(in). Also known as: 2-oxoglutarate:hydrogen symporter activity, 2-oxoglutarate:proton symporter activity, alpha-ketoglutarate:hydrogen symporter activity